{
  "gene_name": "Laminin subunit alpha-3",
  "gene": "UniProtKB:Q16787",
  "term_id": "GO:0005886",
  "term_label": "plasma membrane",
  "gene_symbol": "LAMA3"
}